melanocyte-stimulating hormone secretion [GO:0036160] (biological process) Definition: The regulated release of a melanocyte-stimulating hormone, any of a group of peptide hormones that are produced by cells in the intermediate lobe of the pituitary gland, and stimulate the production of melanin to increase pigmentation. Also known as: MSH secretion Sources: GOC:cjm, Wikipedia:Melanocyte-stimulating_hormone Relationships: is a type of GO:0030072